{
  "gene": "UniProtKB:Q96LR2",
  "term_id": "UNKNOWN:0003",
  "term_label": "Unknown cellular component",
  "gene_name": "Leucine rich adaptor protein 1",
  "gene_symbol": "LURAP1"
}